{
  "term_id": "GO:0090263",
  "term_label": "positive regulation of canonical Wnt signaling pathway",
  "gene_name": "Casein kinase I isoform gamma-2",
  "gene_symbol": "CSNK1G2",
  "gene": "UniProtKB:P78368"
}